{
  "gene_name": "Metalloreductase STEAP2",
  "gene_symbol": "STEAP2",
  "term_label": "cupric reductase (NADH) activity",
  "gene": "UniProtKB:Q8NFT2",
  "term_id": "GO:0008823"
}